{
  "term_label": "glucose-6-phosphatase activity",
  "gene": "UniProtKB:Q9NQR9",
  "term_id": "GO:0004346",
  "gene_name": "Glucose-6-phosphatase 2",
  "gene_symbol": "G6PC2"
}